{
  "gene": "UniProtKB:Q9Y6Q9",
  "gene_name": "Nuclear receptor coactivator 3",
  "term_label": "transcription coactivator activity",
  "term_id": "GO:0003713",
  "gene_symbol": "NCOA3"
}